{
  "term_id": "GO:0061608",
  "gene": "UniProtKB:O15397",
  "gene_symbol": "IPO8",
  "term_label": "nuclear import signal receptor activity",
  "gene_name": "Importin-8"
}